positive regulation of vascular endothelial growth factor signaling pathway [GO:1900748] (biological process) Definition: Any process that activates or increases the frequency, rate or extent of vascular endothelial growth factor signaling pathway. Also known as: activation of VEGF signaling, activation of VEGF-activated signaling pathway, activation of vascular endothelial growth factor signalling pathway, positive regulation of VEGF signaling, positive regulation of VEGF-activated signaling pathway, positive regulation of vascular endothelial growth factor signalling pathway, up regulation of VEGF signaling, up regulation of VEGF-activated signaling pathway, up regulation of vascular endothelial growth factor signaling pathway, up regulation of vascular endothelial growth factor signalling pathway, up-regulation of VEGF signaling, up-regulation of VEGF-activated signaling pathway, up-regulation of vascular endothelial growth factor signaling pathway, up-regulation of vascular endothelial growth factor signalling pathway, upregulation of VEGF signaling, upregulation of VEGF-activated signaling pathway, upregulation of vascular endothelial growth factor signaling pathway, upregulation of vascular endothelial growth factor signalling pathway, activation of vascular endothelial growth factor signaling pathway Sources: GOC:TermGenie Relationships: is a type of positive regulation of signal transduction [GO:0009967]; is_a regulation of vascular endothelial growth factor signaling pathway [GO:1900746]; positively regulates vascular endothelial growth factor signaling pathway [GO:0038084]